{
  "gene_name": "Zinc finger protein 175",
  "gene": "UniProtKB:Q9Y473",
  "gene_symbol": "ZNF175",
  "term_id": "UNKNOWN:0002",
  "term_label": "Unknown biological process"
}